{
  "term_id": "UNKNOWN:0001",
  "term_label": "Unknown molecular function",
  "gene_name": "Ras association domain-containing protein 10",
  "gene_symbol": "RASSF10",
  "gene": "UniProtKB:A6NK89"
}